CAAX-protein geranylgeranyltransferase complex [GO:0005953] (cellular component) Relationships: is a type of intracellular protein-containing complex [GO:0140535]; is a type of transferase complex [GO:1990234] Definition: A heterodimeric enzyme, composed of an alpha and a beta subunit. Participates in the post-translational C-terminal modification of several small GTPases, allowing their targeting to the membrane. References: PMID:9781874